nickel cation binding [GO:0016151] (molecular function) Relationships: is a type of transition metal ion binding [GO:0046914] Sources: GOC:ai Also known as: Ni binding, nickel binding Definition: Binding to a nickel (Ni) cation.